macrophage homeostasis [GO:0061519] (BP) Definition: The process of regulating the proliferation and elimination of macrophage cells such that the total number of myeloid cells within a whole or part of an organism is stable over time in the absence of an outside stimulus. References: PMID:21727904 Sources: GOC:dph Relationships: is a type of GO:0001776; is a type of GO:0002262